positive regulation of myeloid leukocyte mediated immunity [GO:0002888] (biological process) Also known as: up regulation of myeloid leukocyte mediated immunity, up-regulation of myeloid leukocyte mediated immunity, upregulation of myeloid leukocyte mediated immunity, activation of myeloid leukocyte mediated immunity, stimulation of myeloid leukocyte mediated immunity Relationships: is a type of positive regulation of leukocyte mediated immunity [GO:0002705]; is a type of regulation of myeloid leukocyte mediated immunity [GO:0002886]; positively regulates myeloid leukocyte mediated immunity [GO:0002444] Subtypes: GO:0001805, positive regulation of myeloid dendritic cell cytokine production [GO:0002735], positive regulation of type II hypersensitivity [GO:0002894], GO:0043311, positive regulation of neutrophil degranulation [GO:0043315], positive regulation of neutrophil mediated cytotoxicity [GO:0070960], positive regulation of basophil degranulation [GO:1903583], positive regulation of microglial cell mediated cytotoxicity [GO:1904151] Sources: GOC:add Definition: Any process that activates or increases the frequency, rate, or extent of myeloid leukocyte mediated immunity.